cadmium ion binding [GO:0046870] (molecular function) Relationships: is a type of transition metal ion binding [GO:0046914] Also known as: copper/cadmium binding, Cd ion binding, cadmium binding Sources: GOC:ai Definition: Binding to a cadmium ion (Cd).